regulation of natural killer cell apoptotic process [GO:0070247] (biological process) Definition: Any process that modulates the occurrence or rate of natural killer cell death by apoptotic process. Sources: GOC:add, GOC:mtg_apoptosis, ISBN:0781765196 Also known as: regulation of NK cell apoptosis, regulation of natural killer cell apoptosis Relationships: is a type of regulation of lymphocyte apoptotic process [GO:0070228]; regulates natural killer cell apoptotic process [GO:0070246] Subtypes: negative regulation of natural killer cell apoptotic process [GO:0070248], positive regulation of natural killer cell apoptotic process [GO:0070249]